{
  "gene_name": "Small integral membrane protein 44",
  "term_id": "UNKNOWN:0001",
  "gene_symbol": "SMIM44",
  "gene": "UniProtKB:A0A286YF18",
  "term_label": "Unknown molecular function"
}